encapsulin nanocompartment [GO:0140737] (cellular component) Definition: Intracellular non-membrane bound organelle, consisting of proteinaceous polyhedral shells that encapsulate enzymes, protecting the contents from their surrounding milieu and/or the milieu from reactants in their interior. The self-assembling, 25-42 nm nanocompartment shell, unlike larger bacterial microcompartments, is made of only one protein, and has only a few proteins inside. Shells about vary from about 25-42 nm in diameter. The shell protein has an HK97-like fold and probably evolved from a viral protein. Artificial encapsulin nanocompartments can be expressed and filled with cargo proteins for biotechnological uses. They are found in many bacterial and a few archaeal phyla. Also known as: protein nanocompartment Relationships: is a type of intracellular membraneless organelle [GO:0043232] References: PMID:32918485